{
  "term_label": "killing of cells of another organism",
  "term_id": "GO:0031640",
  "gene_name": "Beta-defensin 123",
  "gene_symbol": "DEFB123",
  "gene": "UniProtKB:Q8N688"
}